{
  "term_id": "GO:0000978",
  "gene_name": "Myogenin",
  "term_label": "RNA polymerase II cis-regulatory region sequence-specific DNA binding",
  "gene_symbol": "MYOG",
  "gene": "UniProtKB:P15173"
}